{
  "gene": "UniProtKB:P0CG31",
  "term_id": "GO:0000978",
  "term_label": "RNA polymerase II cis-regulatory region sequence-specific DNA binding",
  "gene_name": "Putative zinc finger protein 286B",
  "gene_symbol": "ZNF286B"
}